positive regulation of cell maturation [GO:1903431] (biological process) Definition: Any process that activates or increases the frequency, rate or extent of cell maturation. References: PMID:17459944 Sources: GOC:TermGenie, GO_REF:0000058 Also known as: up regulation of cell maturation, up-regulation of cell maturation, upregulation of cell maturation, activation of cell maturation, activation of functional differentiation, positive regulation of functional differentiation, up regulation of functional differentiation, up-regulation of functional differentiation, upregulation of functional differentiation Relationships: is_a positive regulation of cell development [GO:0010720]; is a type of regulation of cell maturation [GO:1903429]; positively regulates cell maturation [GO:0048469] Subtypes: positive regulation of neuron maturation [GO:0014042], positive regulation of bicoid mRNA localization [GO:0045854], positive regulation of oocyte maturation [GO:1900195], positive regulation of sperm capacitation [GO:1902492], GO:1902892